{
  "gene_name": "Chorionic somatomammotropin hormone 1",
  "gene": "UniProtKB:P0DML2",
  "term_id": "GO:0005615",
  "term_label": "extracellular space",
  "gene_symbol": "CSH1"
}